{
  "gene_name": "Protein transport protein Sec24A",
  "gene": "UniProtKB:O95486",
  "gene_symbol": "SEC24A",
  "term_label": "endoplasmic reticulum exit site",
  "term_id": "GO:0070971"
}